{
  "gene_name": "Mitochondrial fission 1 protein",
  "term_id": "GO:0008289",
  "gene_symbol": "FIS1",
  "gene": "UniProtKB:Q9Y3D6",
  "term_label": "lipid binding"
}